positive regulation of immune complex clearance by monocytes and macrophages [GO:0090265] (biological process) Sources: GOC:BHF Relationships: is a type of positive regulation of immune effector process [GO:0002699]; is a type of regulation of immune complex clearance by monocytes and macrophages [GO:0090264]; positively regulates immune complex clearance by monocytes and macrophages [GO:0002436] Definition: Any process that increases the rate, frequency, or extent of the process of immune complex clearance by monocytes or macrophages.